{
  "gene_name": "Outer dynein arm-docking complex subunit 4",
  "gene": "UniProtKB:Q96NG3",
  "term_label": "Unknown molecular function",
  "term_id": "UNKNOWN:0001",
  "gene_symbol": "ODAD4"
}